{
  "gene": "UniProtKB:Q8TF08",
  "term_id": "GO:0045277",
  "gene_symbol": "COX7B2",
  "gene_name": "Cytochrome c oxidase subunit 7B2, mitochondrial",
  "term_label": "respiratory chain complex IV"
}